mannosamine biosynthetic process [GO:0046347] (BP) Relationships: is_a GO:0046349 Sources: GOC:curators Definition: The chemical reactions and pathways resulting in the formation of mannosomine, 2-amino-2-deoxymannose; the D-isomer is a constituent of neuraminic acids as well as mucolipids and mucoproteins. Also known as: mannosamine anabolism, mannosamine biosynthesis, mannosamine formation, mannosamine synthesis Subtypes: N-acetylmannosamine biosynthetic process [GO:0006052]